{
  "term_id": "UNKNOWN:0003",
  "gene": "UniProtKB:Q9P104",
  "term_label": "Unknown cellular component",
  "gene_name": "Docking protein 5",
  "gene_symbol": "DOK5"
}